{
  "gene_symbol": "AATF",
  "gene_name": "Protein AATF",
  "gene": "UniProtKB:Q9NY61",
  "term_label": "nucleolus",
  "term_id": "GO:0005730"
}